{
  "gene_symbol": "POLG",
  "gene_name": "DNA polymerase subunit gamma-1",
  "term_id": "GO:0003887",
  "gene": "UniProtKB:P54098",
  "term_label": "DNA-directed DNA polymerase activity"
}